lateral element assembly [GO:0051878] (biological process) Definition: The cell cycle process in which lateral elements are formed. Axial elements form a proteinaceous core between the two sister chromatids of each chromosome; the two axial elements then connect along their entire lengths by fine fibers known as transverse filaments, forming the lateral elements. References: PMID:11463847 Relationships: is a type of GO:0022607; is a type of GO:1903046; is part of synaptonemal complex assembly [GO:0007130]